cyclase regulator activity [GO:0010851] (MF) Subtypes: cyclase inhibitor activity [GO:0010852], GO:0010853, adenylate cyclase regulator activity [GO:0010854], GO:0030249 Relationships: is a type of enzyme regulator activity [GO:0030234]; regulates cyclase activity [GO:0009975] Definition: Binds to and modulates the activity of an enzyme that catalyzes a ring closure reaction. Sources: GOC:dph, GOC:tb